{
  "gene_name": "Heat shock-related 70 kDa protein 2",
  "term_label": "nucleus",
  "gene_symbol": "HSPA2",
  "term_id": "GO:0005634",
  "gene": "UniProtKB:P54652"
}